{
  "gene_symbol": "GAB1",
  "term_label": "cytoplasm",
  "gene_name": "GRB2-associated-binding protein 1",
  "gene": "UniProtKB:Q13480",
  "term_id": "GO:0005737"
}